{
  "term_label": "fibronectin binding",
  "gene_symbol": "ITGB3",
  "gene": "UniProtKB:P05106",
  "term_id": "GO:0001968",
  "gene_name": "Integrin beta-3"
}